{
  "term_label": "plasma membrane",
  "gene": "UniProtKB:A0A0A6YYD4",
  "gene_name": "T cell receptor beta variable 13",
  "gene_symbol": "TRBV13",
  "term_id": "GO:0005886"
}